{
  "gene": "UniProtKB:G2XKQ0",
  "term_label": "ubiquitin-like protein ligase binding",
  "term_id": "GO:0044389",
  "gene_symbol": "SUMO1P1",
  "gene_name": "Small ubiquitin-related modifier 5"
}